{
  "term_label": "Unknown molecular function",
  "gene_name": "Myelin-associated oligodendrocyte basic protein",
  "gene": "UniProtKB:Q13875",
  "term_id": "UNKNOWN:0001",
  "gene_symbol": "MOBP"
}